cystathionine beta-synthase activity [GO:0004122] (molecular function) Definition: Catalysis of the reaction: L-serine + L-homocysteine = cystathionine + H2O. Also known as: L-serine hydro-lyase (adding homocysteine), L-serine hydro-lyase (adding homocysteine; L-cystathionine-forming), beta-thionase activity, methylcysteine synthase activity, serine sulfhydrase activity, serine sulfhydrylase activity Relationships: is a type of GO:0016836 Sources: EC:4.2.1.22